{
  "gene_name": "Telomere repeats-binding bouquet formation protein 1",
  "term_label": "meiotic attachment of telomere to nuclear envelope",
  "gene_symbol": "TERB1",
  "gene": "UniProtKB:Q8NA31",
  "term_id": "GO:0070197"
}